{
  "gene_name": "OCIA domain-containing protein 2",
  "term_label": "Unknown molecular function",
  "term_id": "UNKNOWN:0001",
  "gene_symbol": "OCIAD2",
  "gene": "UniProtKB:Q56VL3"
}